{
  "term_id": "UNKNOWN:0002",
  "gene_symbol": "OR4K5",
  "gene_name": "Olfactory receptor 4K5",
  "term_label": "Unknown biological process",
  "gene": "UniProtKB:Q8NGD3"
}